{
  "gene": "UniProtKB:Q9H841",
  "term_id": "GO:0015693",
  "term_label": "magnesium ion transport",
  "gene_name": "NIPA-like protein 2",
  "gene_symbol": "NIPAL2"
}